{
  "term_label": "heme binding",
  "term_id": "GO:0020037",
  "gene": "UniProtKB:A0A087X1C5",
  "gene_name": "Putative cytochrome P450 2D7",
  "gene_symbol": "CYP2D7"
}